{
  "gene": "UniProtKB:P17213",
  "gene_name": "Bactericidal permeability-increasing protein",
  "gene_symbol": "BPI",
  "term_id": "GO:0005615",
  "term_label": "extracellular space"
}